5-phosphoribose 1-diphosphate biosynthetic process [GO:0006015] (biological process) Also known as: 5-phosphoribose 1-diphosphate anabolism, 5-phosphoribose 1-diphosphate biosynthesis, 5-phosphoribose 1-diphosphate formation, 5-phosphoribose 1-diphosphate synthesis, 5-phosphoribosyl-1-pyrophosphate biosynthesis, 5-phosphoribosyl-1-pyrophosphate biosynthetic process, PRPP biosynthetic process Sources: GOC:ai Relationships: is a type of GO:0046390; is a type of 5-phosphoribose 1-diphosphate metabolic process [GO:0046391] Definition: The chemical reactions and pathways resulting in the formation of 5-phosphoribose 1-diphosphate, also known as 5-phosphoribosyl-1-pyrophosphate.